{
  "term_label": "transmembrane transporter binding",
  "term_id": "GO:0044325",
  "gene": "UniProtKB:Q9NZI2",
  "gene_name": "Kv channel-interacting protein 1",
  "gene_symbol": "KCNIP1"
}